olfactory placode maturation [GO:0071700] (biological process) Definition: A developmental process, independent of morphogenetic (shape) change, that is required for the olfactory placode to attain its fully functional state. The olfactory placode is a thickening of the neural ectoderm in the head region of the vertebrate embryo which develops into the olfactory region of the nasal cavity. Relationships: is a type of anatomical structure maturation [GO:0071695]; BFO_0000050 olfactory placode development [GO:0071698] Sources: GOC:mah